{
  "term_label": "extracellular space",
  "gene_name": "Pulmonary surfactant-associated protein D",
  "gene_symbol": "SFTPD",
  "term_id": "GO:0005615",
  "gene": "UniProtKB:P35247"
}